{
  "gene": "UniProtKB:P37287",
  "gene_name": "Phosphatidylinositol N-acetylglucosaminyltransferase subunit A",
  "gene_symbol": "PIGA",
  "term_id": "GO:0017176",
  "term_label": "phosphatidylinositol N-acetylglucosaminyltransferase activity"
}